{
  "term_label": "RNA binding",
  "gene_name": "RNA-binding protein 33",
  "gene": "UniProtKB:Q96EV2",
  "gene_symbol": "RBM33",
  "term_id": "GO:0003723"
}